citrate:2-oxoglutarate antiporter activity [GO:0180056] (molecular function) Relationships: is a type of alpha-ketoglutarate transmembrane transporter activity [GO:0015139]; is a type of antiporter activity [GO:0015297]; is a type of citrate secondary active transmembrane transporter activity [GO:0071913] Definition: Enables the transfer of a solute or solutes from one side of a membrane to the other according to the reaction: citrate(out) + 2-oxogluarate(in) = citrate(in) + 2-oxogluarat(out). References: PMID:20371607